{
  "gene": "UniProtKB:A6NNM3",
  "term_label": "benzodiazepine receptor binding",
  "term_id": "GO:0030156",
  "gene_symbol": "RIMBP3B",
  "gene_name": "RIMS-binding protein 3B"
}